{
  "gene_name": "C-X-C motif chemokine 10",
  "term_label": "neutrophil chemotaxis",
  "gene_symbol": "CXCL10",
  "term_id": "GO:0030593",
  "gene": "UniProtKB:P02778"
}